{
  "term_label": "regulation of transcription by RNA polymerase II",
  "gene_symbol": "RAX",
  "term_id": "GO:0006357",
  "gene": "UniProtKB:Q9Y2V3",
  "gene_name": "Retinal homeobox protein Rx"
}